{
  "term_id": "GO:0005634",
  "gene_name": "T-box transcription factor TBX4",
  "gene": "UniProtKB:P57082",
  "term_label": "nucleus",
  "gene_symbol": "TBX4"
}